{
  "term_id": "GO:0043161",
  "gene": "UniProtKB:P28066",
  "gene_name": "Proteasome subunit alpha type-5",
  "gene_symbol": "PSMA5",
  "term_label": "proteasome-mediated ubiquitin-dependent protein catabolic process"
}